meiotic DNA recombinase assembly involved in meiotic gene conversion [GO:0010773] (biological process) Relationships: is a type of GO:0000707; is part of meiotic gene conversion [GO:0006311] Sources: GOC:dph, GOC:tb Definition: The aggregation, arrangement and bonding together of strand exchange proteins (recombinases) to form higher order oligomers on single-stranded DNA resulting in meiotic gene conversion. Meiotic gene conversion is the cell cycle process in which genetic information is transferred from one helix to another.